{
  "term_id": "GO:1990756",
  "gene": "UniProtKB:Q0D2K2",
  "term_label": "ubiquitin-like ligase-substrate adaptor activity",
  "gene_symbol": "KLHL30",
  "gene_name": "Kelch-like protein 30"
}